{
  "gene": "UniProtKB:P01137",
  "gene_symbol": "TGFB1",
  "term_id": "GO:0030154",
  "gene_name": "Transforming growth factor beta-1 proprotein",
  "term_label": "cell differentiation"
}